{
  "gene_name": "Triosephosphate isomerase",
  "term_id": "GO:0019563",
  "term_label": "glycerol catabolic process",
  "gene_symbol": "TPI1",
  "gene": "UniProtKB:P60174"
}